{
  "term_label": "natural killer cell activation involved in immune response",
  "term_id": "GO:0002323",
  "gene_name": "Interferon omega-1",
  "gene_symbol": "IFNW1",
  "gene": "UniProtKB:P05000"
}